{
  "gene": "UniProtKB:O43439",
  "term_id": "GO:0003714",
  "gene_name": "Protein CBFA2T2",
  "gene_symbol": "CBFA2T2",
  "term_label": "transcription corepressor activity"
}